medulla oblongata maturation [GO:0021582] (BP) Relationships: is a type of anatomical structure maturation [GO:0071695]; is part of GO:0021550; is part of hindbrain maturation [GO:0021578] Definition: A developmental process, independent of morphogenetic (shape) change, that is required for the medulla oblongata to attain its fully functional state. The medulla oblongata lies directly above the spinal cord and controls vital autonomic functions such as digestion, breathing and the control of heart rate. Sources: GOC:cls, GOC:dgh, GOC:dph, GOC:jid, GO_REF:0000021 Also known as: medulla maturation, myelencephalon maturation